{
  "term_id": "GO:0008361",
  "gene_symbol": "ARHGAP5",
  "term_label": "regulation of cell size",
  "gene": "UniProtKB:Q13017",
  "gene_name": "Rho GTPase-activating protein 5"
}